regulation of skeletal muscle contraction by chemo-mechanical energy conversion [GO:0014862] (biological process) Subtypes: regulation of the force of skeletal muscle contraction [GO:0014728], GO:0014729 Relationships: is a type of regulation of skeletal muscle contraction [GO:0014819] Definition: Any process that modulates the frequency, rate or extent of skeletal muscle contraction by regulating force and velocity of shortening. The force of skeletal muscle contraction is produced by acto-myosin interaction processes through formation of cross bridges. The shortening leads to reduction of length of muscle fiber and sarcomeres. Sources: GOC:mtg_muscle